regulation of maintenance of mitotic sister chromatid cohesion, telomeric [GO:1904907] (biological process) References: PMID:26373281 Sources: GOC:BHF, GOC:BHF_telomere, GOC:TermGenie, GOC:rph, GO_REF:0000058 Also known as: regulation of maintenance of mitotic sister chromatin cohesion at telomere, regulation of maintenance of sister chromatin cohesion at telomere at mitosis, regulation of maintenance of telomeric mitotic sister chromatin cohesion Relationships: is a type of regulation of maintenance of mitotic sister chromatid cohesion [GO:0034182]; regulates maintenance of mitotic sister chromatid cohesion, telomeric [GO:0099403] Definition: Any process that modulates the frequency, rate or extent of maintenance of mitotic sister chromatid cohesion, telomeric. Subtypes: negative regulation of maintenance of mitotic sister chromatid cohesion, telomeric [GO:1904908], GO:1904909